tRNA transcription by RNA polymerase III [GO:0042797] (biological process) Also known as: tRNA transcription from Pol III promoter, tRNA transcription from RNA polymerase III promoter Definition: The synthesis of transfer RNA (tRNA) from a DNA template by RNA polymerase III (Pol III), originating at a Pol III promoter. Relationships: is a type of transcription by RNA polymerase III [GO:0006383]; is a type of tRNA transcription [GO:0009304] Sources: GOC:jl, ISBN:0321000382